{
  "gene": "UniProtKB:Q96IZ5",
  "gene_name": "RNA-binding protein 41",
  "term_label": "mRNA splicing, via spliceosome",
  "term_id": "GO:0000398",
  "gene_symbol": "RBM41"
}